{
  "gene_symbol": "IGKV1D-33",
  "term_id": "GO:0019814",
  "term_label": "immunoglobulin complex",
  "gene": "UniProtKB:P01593",
  "gene_name": "Immunoglobulin kappa variable 1D-33"
}